negative regulation of cardiac neural crest cell migration involved in outflow tract morphogenesis [GO:1905311] (biological process) Relationships: is a type of negative regulation of cell migration [GO:0030336]; is a type of regulation of cardiac neural crest cell migration involved in outflow tract morphogenesis [GO:1905310]; negatively regulates GO:0003253 Definition: Any process that stops, prevents or reduces the frequency, rate or extent of cardiac neural crest cell migration involved in outflow tract morphogenesis. References: PMID:17628518 Sources: GOC:BHF, GOC:TermGenie, GOC:rl, GO_REF:0000058 Also known as: down regulation of cardiac neural crest cell migration involved in outflow tract morphogenesis, down-regulation of cardiac neural crest cell migration involved in outflow tract morphogenesis, downregulation of cardiac neural crest cell migration involved in outflow tract morphogenesis, inhibition of cardiac neural crest cell migration involved in outflow tract morphogenesis